murein tripeptide carboxypeptidase activity [GO:0061473] (molecular function) Definition: Catalysis of the reaction: L-alanyl-gamma-D-glutamyl-meso-diaminoheptanedioate (murein tripeptide) + H2O = L-alanyl-D-glutamate + meso-2,6-diaminoheptanedioate. Relationships: is_a metallocarboxypeptidase activity [GO:0004181] References: PMID:22970852 Sources: RHEA:28398